O-acyl-L-carnitine transmembrane transport [GO:1902616] (biological process) Also known as: O-acylcarnitine transmembrane transport Sources: GOC:TermGenie, GOC:pr, GO_REF:0000069 Relationships: is a type of quaternary ammonium group transport [GO:0015697]; is a type of transmembrane transport [GO:0055085] Definition: The process in which O-acyl-L-carnitine is transported across a membrane.